{
  "gene": "UniProtKB:P23258",
  "gene_name": "Tubulin gamma-1 chain",
  "term_id": "GO:0000931",
  "term_label": "gamma-tubulin ring complex",
  "gene_symbol": "TUBG1"
}